{
  "gene": "UniProtKB:Q9BRG2",
  "gene_symbol": "SH2D3A",
  "term_label": "Unknown cellular component",
  "gene_name": "SH2 domain-containing protein 3A",
  "term_id": "UNKNOWN:0003"
}